pheromone binding [GO:0005550] (molecular function) Sources: GOC:ai Relationships: is a type of odorant binding [GO:0005549] Definition: Binding to a pheromone, a substance, or characteristic mixture of substances, that is secreted and released by an organism and detected by a second organism of the same or a closely related species, in which it causes a specific reaction, such as a definite behavioral reaction or a developmental process.